{
  "gene_symbol": "ATL2",
  "term_id": "UNKNOWN:0003",
  "gene": "UniProtKB:Q8NHH9",
  "term_label": "Unknown cellular component",
  "gene_name": "Atlastin-2"
}